myeloid leukocyte cytokine production [GO:0061082] (biological process) Note: Note that this term is in the subset of terms that should not be used for direct gene product annotation. Instead, select one of the 'regulation' children terms. Subtypes: myeloid dendritic cell cytokine production [GO:0002372], GO:0010934, GO:0032762 Relationships: is a type of GO:0002367 Sources: GOC:dph Definition: Any process that contributes to cytokine production by a myeloid cell. Regulation: positively regulated by GO:0061081